regulation of glycogen catabolic process [GO:0005981] (biological process) Sources: GOC:go_curators Definition: Any process that modulates the frequency, rate or extent of the chemical reactions and pathways resulting in the breakdown of glycogen. Relationships: is a type of GO:0043470; is a type of regulation of glycogen metabolic process [GO:0070873]; regulates glycogen catabolic process [GO:0005980] Also known as: regulation of glycogen breakdown, regulation of glycogen catabolism, regulation of glycogen degradation, regulation of glycogenolysis Subtypes: negative regulation of glycogen catabolic process [GO:0045818], GO:0045819